CDP-diacylglycerol-inositol 3-phosphatidyltransferase activity [GO:0003881] (molecular function) Also known as: phosphatidylinositol synthase activity, CDP diglyceride-inositol phosphatidyltransferase activity, CDP-DG:inositol transferase activity, CDP-diacylglycerol--inositol phosphatidyltransferase activity, CDP-diacylglycerol:myo-inositol 3-phosphatidyltransferase activity, CDP-diacylglycerol:myo-inositol-3-phosphatidyltransferase activity, CDP-diglyceride-inositol transferase activity, CDP-diglyceride:inositol transferase activity, CDPdiacylglycerol-inositol 3-phosphatidyltransferase activity, cytidine 5'-diphospho-1,2-diacyl-sn-glycerol:myo-inositol 3-phosphatidyltransferase activity, cytidine diphosphodiglyceride-inositol phosphatidyltransferase activity, cytidine diphosphoglyceride-inositol phosphatidyltransferase activity, cytidine diphosphoglyceride-inositol transferase activity Sources: EC:2.7.8.11, RHEA:11580 Relationships: is a type of CDP-alcohol phosphatidyltransferase activity [GO:0017169] Definition: Catalysis of the reaction: myo-inositol + CDP-diacylglycerol = 1-phosphatidyl-1D-myo-inositol + CMP + H+.